regulation of Cdc42 protein signal transduction [GO:0032489] (biological process) Definition: Any process that modulates the frequency, rate or extent of Cdc42 protein signal transduction. Sources: GOC:mah Relationships: is a type of regulation of Rho protein signal transduction [GO:0035023]; regulates GO:0032488